internal side of mycolate outer membrane [GO:0098569] (cellular component) Definition: The side of the mycolate outer membrane that faces the cell wall peptidoglycan. It is rich in long-chain mycolic acids (hydroxylated branched-chain fatty acids) that are covalently linked to the cell wall peptidoglycan via an arabinogalactan network. References: PMID:18316738, PMID:18567661 Sources: GOC:dos Relationships: is a type of side of membrane [GO:0098552]